{
  "term_id": "GO:0030198",
  "term_label": "extracellular matrix organization",
  "gene": "UniProtKB:Q5TAT6",
  "gene_name": "Collagen alpha-1(XIII) chain",
  "gene_symbol": "COL13A1"
}